BtuCD complex [GO:1990193] (cellular component) References: PMID:22569249 Sources: GOC:bhm Also known as: BtuC-BtuD complex, cobalamin transport complex, core subunit, vitamin B12 transport complex, core subunit Relationships: is a type of ATP-binding cassette (ABC) transporter complex [GO:0043190] Definition: Protein complex involved in cobalamin (vitamin B12) transport through the plasma membrane. In E. coli, the complex is a tetramer and consists of the cytoplasmic ATPase BtuD homodimer together with the transmembrane BtuC homodimer.